{
  "term_label": "regulation of transcription by RNA polymerase II",
  "gene_symbol": "ERG",
  "gene": "UniProtKB:P11308",
  "term_id": "GO:0006357",
  "gene_name": "Transcriptional regulator ERG"
}